thermotaxis [GO:0043052] (BP) Definition: The directed movement of a motile cell or organism in response to a temperature gradient. Movement may be towards either a higher or lower temperature. Sources: GOC:cab1, WB_REF:cgc467 Also known as: taxis in response to temperature stimulus Relationships: is a type of response to temperature stimulus [GO:0009266]; is a type of taxis [GO:0042330]